{
  "gene_symbol": "SFTPD",
  "gene": "UniProtKB:P35247",
  "term_id": "GO:0043129",
  "gene_name": "Pulmonary surfactant-associated protein D",
  "term_label": "surfactant homeostasis"
}